fatty-acyl-CoA metabolic process [GO:0035337] (biological process) Subtypes: GO:0035336, very long-chain fatty-acyl-CoA metabolic process [GO:0036111], medium-chain fatty-acyl-CoA metabolic process [GO:0036112], fatty-acyl-CoA catabolic process [GO:0036115], GO:0046949, branched-chain alpha-keto acid decarboxylation to branched-chain acyl-CoA [GO:0120552], GO:1902192, 3-methylbut-2-enoyl-CoA(4-) metabolic process [GO:1902198], propionyl-CoA metabolic process [GO:1902858] Also known as: fatty acyl CoA metabolic process, fatty-acyl-CoA metabolism Relationships: is a type of acyl-CoA metabolic process [GO:0006637]; is a type of fatty acid derivative metabolic process [GO:1901568] Sources: ISBN:0198506732 Definition: The chemical reactions and pathways involving a fatty-acyl-CoA, any derivative of coenzyme A in which the sulfhydryl group is in thiolester linkage with a fatty-acyl group.